metanephric podocyte cell fate commitment [GO:0072250] (BP) Sources: GOC:mtg_kidney_jan10 Relationships: is a type of podocyte cell fate commitment [GO:0072149]; is a type of metanephric glomerular epithelial cell fate commitment [GO:0072315]; is part of metanephric podocyte differentiation [GO:0072248] Definition: The process in which the developmental fate of a cell becomes restricted such that it will develop into a metanephric glomerular visceral epithelial cell. A metanephric glomerular visceral epithelial cell is a specialized epithelial cell that contains 'feet' that interdigitate with the 'feet' of other glomerular epithelial cells in the metanephros. Also known as: metanephric glomerular visceral epithelial cell fate commitment